{
  "term_id": "GO:0006182",
  "gene_symbol": "NPPA",
  "gene": "UniProtKB:P01160",
  "gene_name": "Natriuretic peptides A",
  "term_label": "cGMP biosynthetic process"
}